positive regulation of bicellular tight junction assembly [GO:1903348] (biological process) Relationships: is a type of positive regulation of cell junction assembly [GO:1901890]; is a type of regulation of bicellular tight junction assembly [GO:2000810]; positively regulates bicellular tight junction assembly [GO:0070830] References: PMID:25050009 Sources: GOC:TermGenie, GOC:jz, GO_REF:0000058 Definition: Any process that activates or increases the frequency, rate or extent of tight junction assembly. Also known as: positive regulation of tight junction formation, up regulation of tight junction assembly, up regulation of tight junction formation, up-regulation of tight junction assembly, up-regulation of tight junction formation, upregulation of tight junction assembly, upregulation of tight junction formation, activation of tight junction assembly, activation of tight junction formation